half bridge of spindle pole body [GO:0005825] (cellular component) Relationships: is a type of cellular anatomical structure [GO:0110165]; is part of spindle pole body [GO:0005816] Subtypes: half bridge of mitotic spindle pole body [GO:0061496] Definition: Structure adjacent to the plaques of the spindle pole body. Sources: ISBN:0879693568